histidinol-phosphate transaminase activity [GO:0004400] (molecular function) Also known as: histidinol-phosphate aminotransferase activity, IAP transaminase activity, L-histidinol phosphate aminotransferase activity, L-histidinol-phosphate:2-oxoglutarate aminotransferase activity, glutamic-imidazoleacetol phosphate transaminase activity, histidine:imidazoleacetol phosphate transaminase activity, histidinol phosphate aminotransferase activity, imidazole acetol-phosphate transaminase activity, imidazoleacetol phosphate transaminase activity, imidazolylacetolphosphate aminotransferase activity, imidazolylacetolphosphate transaminase activity Sources: EC:2.6.1.9 Relationships: is a type of GO:0008483 Definition: Catalysis of the reaction: L-histidinol-phosphate + 2-oxoglutarate = 3-(imidazol-4-yl)-2-oxopropyl phosphate + L-glutamate.